regulation of low-density lipoprotein particle clearance [GO:0010988] (biological process) Subtypes: negative regulation of low-density lipoprotein particle clearance [GO:0010989], positive regulation of low-density lipoprotein particle clearance [GO:1905581] Definition: Any process that modulates the rate, frequency or extent of low-density lipoprotein particle clearance. Low-density lipoprotein particle clearance is the process in which a low-density lipoprotein particle is removed from the blood via receptor-mediated endocytosis and its constituent parts degraded. Sources: GOC:BHF, GOC:dph, GOC:tb Relationships: is a type of regulation of lipoprotein particle clearance [GO:0010984]; regulates low-density lipoprotein particle clearance [GO:0034383]